{
  "term_id": "GO:0019885",
  "term_label": "antigen processing and presentation of endogenous peptide antigen via MHC class I",
  "gene": "UniProtKB:Q03518",
  "gene_name": "Antigen peptide transporter 1",
  "gene_symbol": "TAP1"
}